{
  "term_id": "GO:0006893",
  "gene_symbol": "STXBP5",
  "gene_name": "Syntaxin-binding protein 5",
  "gene": "UniProtKB:Q5T5C0",
  "term_label": "Golgi to plasma membrane transport"
}